{
  "gene": "UniProtKB:Q9UMD9",
  "gene_symbol": "COL17A1",
  "term_id": "GO:0030020",
  "term_label": "extracellular matrix structural constituent conferring tensile strength",
  "gene_name": "Collagen alpha-1(XVII) chain"
}